{
  "gene": "UniProtKB:Q86SY8",
  "gene_symbol": "KTN1-AS1",
  "term_label": "Unknown molecular function",
  "term_id": "UNKNOWN:0001",
  "gene_name": "Putative uncharacterized protein KTN1-AS1"
}